polynucleotide 5'-phosphatase activity [GO:0004651] (molecular function) Sources: EC:3.1.3.33 Definition: Catalysis of the reaction: a 5'-phosphopolynucleotide + H2O = a polynucleotide + phosphate. Relationships: is a type of phosphatase activity [GO:0016791] Also known as: 5'-polynucleotidase activity, polynucleotide 5'-phosphohydrolase activity, polynucleotide 5'-triphosphatase activity